{
  "gene": "UniProtKB:A4QMS7",
  "gene_name": "Cilia- and flagella-associated protein 90",
  "term_label": "Unknown biological process",
  "gene_symbol": "CFAP90",
  "term_id": "UNKNOWN:0002"
}